{
  "gene_symbol": "OR2L2",
  "term_id": "GO:0050911",
  "term_label": "detection of chemical stimulus involved in sensory perception of smell",
  "gene": "UniProtKB:Q8NH16",
  "gene_name": "Olfactory receptor 2L2"
}